heteroduplex formation involved in double-strand break repair via synthesis-dependent strand annealing [GO:0010709] (biological process) Definition: The formation of a stable duplex DNA that contains one strand from each of the two recombining DNA molecules resulting in the error-free repair of a double-strand break without the exchange of adjacent sequences. Relationships: is a type of heteroduplex formation [GO:0030491]; is part of double-strand break repair via synthesis-dependent strand annealing [GO:0045003] Sources: GOC:dph, GOC:tb